oogonium stage [GO:0048158] (biological process) Definition: The stage in mammalian oogenesis when the primordial germ cell is hardly distinguishable from other cortical cells of the ovary. Sources: GOC:jid, GOC:mtg_sensu, ISBN:0198542771 Also known as: mammalian oogenesis stage 1 Relationships: is_a GO:0022605